negative regulation of female gonad development [GO:2000195] (biological process) Sources: GOC:obol Definition: Any process that stops, prevents, or reduces the frequency, rate or extent of female gonad development. Relationships: is a type of GO:1905940; is_a regulation of female gonad development [GO:2000194]; RO_0002212 female gonad development [GO:0008585] Subtypes: negative regulation of progesterone secretion [GO:2000871] Also known as: negative regulation of ovarian development, negative regulation of ovary development